cellular response to reactive oxygen species [GO:0034614] (biological process) Also known as: cellular response to AOS, cellular response to ROI, cellular response to ROS, cellular response to active oxygen species, cellular response to reactive oxidative species, cellular response to reactive oxygen intermediate Relationships: is a type of response to reactive oxygen species [GO:0000302]; is a type of cellular response to oxidative stress [GO:0034599]; is a type of cellular response to oxygen-containing compound [GO:1901701] Subtypes: cellular response to hydrogen peroxide [GO:0070301], cellular response to oxygen radical [GO:0071450], cellular response to singlet oxygen [GO:0071452], cellular response to ozone [GO:0071457] Sources: GOC:mah Definition: Any process that results in a change in state or activity of a cell (in terms of movement, secretion, enzyme production, gene expression, etc.) as a result of a reactive oxygen species stimulus. Reactive oxygen species include singlet oxygen, superoxide, and oxygen free radicals.